deaminase activity [GO:0019239] (molecular function) Sources: GOC:jl Relationships: is a type of hydrolase activity, acting on carbon-nitrogen (but not peptide) bonds [GO:0016810] Subtypes: adenine deaminase activity [GO:0000034], GO:0003726, GO:0004000, cytidine deaminase activity [GO:0004126], GO:0004131, dCMP deaminase activity [GO:0004132], dihydropterin deaminase activity [GO:0004153], glucosamine-6-phosphate deaminase activity [GO:0004342], 1-aminocyclopropane-1-carboxylate deaminase activity [GO:0008660], GO:0008829, diaminohydroxyphosphoribosylaminopyrimidine deaminase activity [GO:0008835], guanine deaminase activity [GO:0008892], dCTP deaminase (dUMP-forming) activity [GO:0033973], isoguanine deaminase activity [GO:0035888], 2'-deoxyadenosine deaminase activity [GO:0046936], GO:0047424, 1-pyrroline-4-hydroxy-2-carboxylate deaminase activity [GO:0047425], adenosine-phosphate deaminase activity [GO:0047623], blasticidin-S deaminase activity [GO:0047711], creatinine deaminase activity [GO:0047790], GO:0047974, GO:0050228, pyrithiamine deaminase activity [GO:0050239], GO:0050270, sepiapterin deaminase activity [GO:0050279], GO:0050540, N6-methyl-AMP deaminase activity [GO:0062154], cAMP deaminase activity [GO:0090612], 5'-deoxyadenosine deaminase activity [GO:0090613], 5'-methylthioadenosine deaminase activity [GO:0090614], GO:0120241 Definition: Catalysis of the removal of an amino group from a substrate, producing a substituted or nonsubstituted ammonia (NH3/NH2R).